{
  "gene": "UniProtKB:Q9NR56",
  "gene_symbol": "MBNL1",
  "term_label": "regulation of RNA splicing",
  "gene_name": "Muscleblind-like protein 1",
  "term_id": "GO:0043484"
}